protein-phosphocysteine-trehalose phosphotransferase system transporter activity [GO:0090589] (molecular function) References: PMID:7608078 Definition: Catalysis of the PEP-dependent, phosphoryl transfer-driven transport of substances across a membrane. The transport happens by catalysis of the reaction: protein S-phosphocysteine + trehalose (out) = protein cysteine + trehalose-6-phosphate (in). Relationships: is a type of protein-phosphocysteine-sugar phosphotransferase activity [GO:0090563]